myosin light chain kinase activity [GO:0004687] (molecular function) Sources: EC:2.7.11.18 Also known as: ATP:myosin-light-chain O-phosphotransferase, myosin light-chain kinase, myosin-light-chain kinase activity, smooth-muscle-myosin-light-chain kinase activity, ATP:myosin-light-chain O-phosphotransferase activity, MLCK, MLCkase activity, STK18, calcium/calmodulin-dependent myosin light chain kinase activity, myosin kinase activity, myosin light chain protein kinase activity, myosin light-chain kinase (phosphorylating), myosin light-chain kinase (phosphorylating) activity, myosin light-chain kinase activity Relationships: is a type of protein serine/threonine kinase activity [GO:0004674] Definition: Catalysis of the reaction: ATP + myosin-light-chain = ADP + myosin-light-chain phosphate.